nascent polypeptide-associated complex binding [GO:1990593] (molecular function) References: PMID:25487825 Relationships: is a type of protein-containing complex binding [GO:0044877] Also known as: NAC binding, NACA binding Definition: Binding to nascent polypeptide-associated complex, a heterodimeric protein complex that can reversibly bind to ribosomes and is located in direct proximity to newly synthesized polypeptide chains as they emerge from the ribosome.